Purkinje myocyte to ventricular cardiac muscle cell communication by electrical coupling [GO:0086055] (BP) Sources: GOC:BHF, GOC:mtg_cardiac_conduct_nov11 Relationships: is a type of GO:0086064; is a type of Purkinje myocyte to ventricular cardiac muscle cell communication [GO:0086068] Definition: The process that mediates signaling interactions between a Purkinje myocyte and a ventricular cardiac muscle cell by transfer of current between their adjacent cytoplasms via intercellular protein channels.